{
  "gene": "UniProtKB:Q6PI47",
  "gene_symbol": "KCTD18",
  "term_label": "Unknown biological process",
  "gene_name": "BTB_POZ domain-containing protein KCTD18",
  "term_id": "UNKNOWN:0002"
}